{
  "gene": "UniProtKB:Q0JRZ9",
  "term_id": "GO:0005905",
  "gene_name": "F-BAR domain only protein 2",
  "term_label": "clathrin-coated pit",
  "gene_symbol": "FCHO2"
}